{
  "term_id": "GO:0034686",
  "gene_name": "Integrin alpha-V",
  "term_label": "integrin alphav-beta8 complex",
  "gene": "UniProtKB:P06756",
  "gene_symbol": "ITGAV"
}